{
  "gene_name": "Cell cycle control protein 50A",
  "gene_symbol": "TMEM30A",
  "term_id": "GO:0005783",
  "gene": "UniProtKB:Q9NV96",
  "term_label": "endoplasmic reticulum"
}